diaminopimelate biosynthetic process [GO:0019877] (biological process) Definition: The chemical reactions and pathways resulting in the formation of diaminopimelate, both as an intermediate in lysine biosynthesis and as a component (as meso-diaminopimelate) of the peptidoglycan of Gram-negative bacterial cell walls. Relationships: is a type of amino acid biosynthetic process [GO:0008652]; is a type of dicarboxylic acid biosynthetic process [GO:0043650]; is a type of fatty acid derivative biosynthetic process [GO:1901570] Sources: GOC:ma, ISBN:0198547684 Also known as: diaminopimelate anabolism, diaminopimelate biosynthesis, diaminopimelate formation, diaminopimelate synthesis